{
  "gene": "UniProtKB:P05160",
  "term_id": "UNKNOWN:0003",
  "term_label": "Unknown cellular component",
  "gene_symbol": "F13B",
  "gene_name": "Coagulation factor XIII B chain"
}